{
  "term_label": "A-type (transient outward) potassium channel activity",
  "term_id": "GO:0005250",
  "gene_name": "Potassium voltage-gated channel subfamily D member 1",
  "gene_symbol": "KCND1",
  "gene": "UniProtKB:Q9NSA2"
}